U7 snRNP [GO:0005683] (CC) Relationships: is a type of GO:0030532 Definition: A ribonucleoprotein complex that contains the U7 snRNA and is required for the 3'-end processing of replication-dependent histone pre-mRNAs. Also known as: snRNP U7 References: PMID:12872004